negative regulation of intracellular sterol transport [GO:0032381] (BP) Subtypes: GO:0032384 Definition: Any process that stops, prevents, or reduces the frequency, rate or extent of the directed movement of sterols within cells. Sources: GOC:mah Relationships: is a type of GO:0032372; is a type of negative regulation of intracellular lipid transport [GO:0032378]; is a type of regulation of intracellular sterol transport [GO:0032380]; RO_0002212 intracellular sterol transport [GO:0032366] Also known as: down regulation of intracellular sterol transport, down-regulation of intracellular sterol transport, downregulation of intracellular sterol transport, inhibition of intracellular sterol transport